{
  "gene": "UniProtKB:Q9BRY0",
  "term_id": "GO:0005886",
  "gene_name": "Zinc transporter ZIP3",
  "term_label": "plasma membrane",
  "gene_symbol": "SLC39A3"
}